formate catabolic process [GO:0042183] (biological process) Also known as: formate breakdown, formate catabolism, formate degradation, formic acid catabolic process, formic acid catabolism Relationships: is a type of formate metabolic process [GO:0015942]; is a type of GO:0072329 Definition: The chemical reactions and pathways resulting in the breakdown of formate, also known as methanoate, the anion HCOO- derived from methanoic (formic) acid. Sources: ISBN:0198506732